locomotory exploration behavior [GO:0035641] (biological process) References: PMID:17151232 Sources: GOC:sart Definition: The specific movement from place to place of an organism in response to a novel environment. Relationships: is a type of locomotory behavior [GO:0007626]; is_a exploration behavior [GO:0035640]